{
  "gene_name": "Neuroligin-4, Y-linked",
  "term_id": "GO:0099634",
  "gene": "UniProtKB:Q8NFZ3",
  "term_label": "postsynaptic specialization membrane",
  "gene_symbol": "NLGN4Y"
}